{
  "term_label": "cell division",
  "gene_symbol": "CDC27",
  "gene": "UniProtKB:P30260",
  "term_id": "GO:0051301",
  "gene_name": "Cell division cycle protein 27 homolog"
}